Fc receptor complex [GO:0032997] (cellular component) Definition: A protein complex composed of a subunit or subunits capable of binding the Fc portion of an immunoglobulin with additional signaling components. The complex functions as a receptor for immunoglobulin. Also known as: immunoglobulin receptor complex, Fc-receptor complex, FcR complex Subtypes: GO:0032998, Fc-alpha receptor I complex [GO:0032999], GO:0033000, GO:0033001 Sources: GOC:add, ISBN:0781735149 Relationships: is_a plasma membrane protein complex [GO:0098797]